plasma membrane-derived photosystem I [GO:0030094] (cellular component) Sources: GOC:jid, GOC:mtg_sensu Also known as: plasma membrane photosystem I Definition: A protein complex located in the plasma membrane-derived thylakoid. The photosystem functions as a light-dependent plastocyanin-ferredoxin oxidoreductase, transferring electrons from plastocyanin to ferredoxin. Examples of this complex are found in bacterial species. Relationships: is a type of photosystem I [GO:0009522]; is a type of plasma membrane protein complex [GO:0098797]; is part of cytoplasm [GO:0005737]; is part of bacterial thylakoid [GO:0030075]